{
  "term_label": "transcription coactivator activity",
  "term_id": "GO:0003713",
  "gene": "UniProtKB:Q969T9",
  "gene_symbol": "WBP2",
  "gene_name": "WW domain-binding protein 2"
}